{
  "term_id": "GO:0005881",
  "term_label": "cytoplasmic microtubule",
  "gene": "UniProtKB:Q6ZUX3",
  "gene_name": "TOG array regulator of axonemal microtubules protein 2",
  "gene_symbol": "TOGARAM2"
}